{
  "term_id": "GO:0035102",
  "term_label": "PRC1 complex",
  "gene": "UniProtKB:Q9BSM1",
  "gene_name": "Polycomb group RING finger protein 1",
  "gene_symbol": "PCGF1"
}